IgG immunoglobulin transcytosis in epithelial cells mediated by FcRn immunoglobulin receptor [GO:0002416] (biological process) Sources: GOC:add, ISBN:0781735149, ISBN:081533642X Also known as: IgG antibody transcytosis in epithelial cells mediated by FcRn immunoglobulin receptor, IgG immunoglobulin transcytosis in epithelial cells mediated by neonatal immunoglobulin receptor Definition: The process of transporting IgG immunoglobulin, via transcytosis using the FcRn (also known as the neonatal Fc receptor; gene name FCGRT), from apical surface of an epithelial cell to the basolateral surface or vice versa depending on the location. This process is used for uptake of IgG from the milk in the gut in rodents, for transplacental transport of IgG from mother to embryo in humans, and for maintenance of a steady-state distribution of IgG across epithelial boundaries in general in adult mammals. Relationships: is a type of immunoglobulin transcytosis in epithelial cells [GO:0002414]